{
  "term_id": "GO:0030619",
  "gene_name": "U1 small nuclear ribonucleoprotein 70 kDa",
  "gene": "UniProtKB:P08621",
  "term_label": "U1 snRNA binding",
  "gene_symbol": "SNRNP70"
}